{
  "term_label": "nucleus",
  "term_id": "GO:0005634",
  "gene_name": "Zinc finger protein 827",
  "gene_symbol": "ZNF827",
  "gene": "UniProtKB:Q17R98"
}